{
  "gene_name": "Ras-related protein Rab-44",
  "gene_symbol": "RAB44",
  "term_label": "vesicle-mediated transport",
  "term_id": "GO:0016192",
  "gene": "UniProtKB:Q7Z6P3"
}